{
  "term_label": "olfactory receptor activity",
  "term_id": "GO:0004984",
  "gene_name": "Olfactory receptor 5W2",
  "gene_symbol": "OR5W2",
  "gene": "UniProtKB:Q8NH69"
}